pyrimidine-containing compound metabolic process [GO:0072527] (biological process) Definition: The chemical reactions and pathways involving a pyrimidine-containing compound, i.e. any compound that contains pyrimidine or a formal derivative thereof. Sources: GOC:mah Also known as: pyrimidine and derivative metabolic process, pyrimidine-containing compound metabolism Relationships: is a type of metabolic process [GO:0008152] Subtypes: GO:0006206, GO:0006213, pyrimidine nucleotide metabolic process [GO:0006220], thiamine-containing compound metabolic process [GO:0042723], pyrimidine-containing compound biosynthetic process [GO:0072528], pyrimidine-containing compound catabolic process [GO:0072529]